{
  "term_label": "Unknown molecular function",
  "term_id": "UNKNOWN:0001",
  "gene_name": "NACHT, LRR and PYD domains-containing protein 12",
  "gene": "UniProtKB:P59046",
  "gene_symbol": "NLRP12"
}